ventral disc dorsal microribbon [GO:0097594] (cellular component) References: PMID:11432808 Sources: GOC:giardia Relationships: is a type of cellular anatomical structure [GO:0110165]; is part of ventral disc [GO:0097597] Definition: Trilaminar structure extending perpendicularly into the cytoplasm along the length of ventral disc microtubules in Giardia species (trophozoite stage). Constituents of dorsal microribbons (also called dorsal ribbons or microribbons) include alpha-coiled-helix proteins approximately 29 to 38 kDa in size. These proteins line the edges of the microribbons but are not found in microtubules. Tubulins are not found in microribbons. Note: Due to the asymmetric nature of the Giardia trophozoite, this term is defined spatially as the trophozoite is viewed from the dorsal side, with the two nuclei dorsal to the ventral disc, and the ventral disc toward the anterior. Also known as: dorsal microribbon, dorsal ribbon, microribbon, ventral disk dorsal microribbon